{
  "term_id": "GO:0031594",
  "gene_symbol": "SYNGR1",
  "term_label": "neuromuscular junction",
  "gene_name": "Synaptogyrin-1",
  "gene": "UniProtKB:O43759"
}